{
  "gene": "UniProtKB:Q9HCU4",
  "term_label": "cell-cell adhesion mediated by cadherin",
  "gene_name": "Cadherin EGF LAG seven-pass G-type receptor 2",
  "term_id": "GO:0044331",
  "gene_symbol": "CELSR2"
}